{
  "term_id": "GO:0008340",
  "gene_name": "5-demethoxyubiquinone hydroxylase, mitochondrial",
  "term_label": "determination of adult lifespan",
  "gene": "UniProtKB:Q99807",
  "gene_symbol": "COQ7"
}